{
  "gene": "UniProtKB:Q96RS0",
  "gene_symbol": "TGS1",
  "term_label": "RNA cap trimethylguanosine synthase activity",
  "gene_name": "Trimethylguanosine synthase",
  "term_id": "GO:0071164"
}